{
  "gene": "UniProtKB:Q96AE4",
  "gene_name": "Far upstream element-binding protein 1",
  "term_label": "regulation of transcription by RNA polymerase II",
  "gene_symbol": "FUBP1",
  "term_id": "GO:0006357"
}